ribonucleoside diphosphate biosynthetic process [GO:0009188] (BP) Also known as: ribonucleoside diphosphate anabolism, ribonucleoside diphosphate biosynthesis, ribonucleoside diphosphate formation, ribonucleoside diphosphate synthesis Definition: The chemical reactions and pathways resulting in the formation of a ribonucleoside diphosphate, a compound consisting of a nucleobase linked to a ribose sugar esterified with diphosphate on the sugar. Subtypes: purine ribonucleoside diphosphate biosynthetic process [GO:0009180], pyrimidine ribonucleoside diphosphate biosynthetic process [GO:0009194] Relationships: is a type of nucleoside diphosphate biosynthetic process [GO:0009133]; is a type of ribonucleoside diphosphate metabolic process [GO:0009185] Sources: GOC:go_curators, ISBN:0198506732